{
  "gene": "UniProtKB:Q9UBL9",
  "gene_name": "P2X purinoceptor 2",
  "term_label": "receptor complex",
  "term_id": "GO:0043235",
  "gene_symbol": "P2RX2"
}